detection of oxidative stress [GO:0070994] (biological process) Definition: The series of events in which a stimulus indicating oxidative stress is received and converted into a molecular signal. Relationships: is a type of response to oxidative stress [GO:0006979] Sources: GOC:mah